{
  "term_label": "Unknown biological process",
  "gene_symbol": "PLA2G3",
  "gene_name": "Group 3 secretory phospholipase A2",
  "term_id": "UNKNOWN:0002",
  "gene": "UniProtKB:Q9NZ20"
}